meiotic spindle pole body [GO:0035974] (cellular component) Definition: The microtubule organizing center that forms as part of the meiotic cell cycle; functionally homologous to the animal cell centrosome. Relationships: is_a spindle pole body [GO:0005816] References: PMID:21775631 Sources: GOC:vw